{
  "gene_name": "MAP kinase-interacting serine_threonine-protein kinase 1",
  "term_id": "GO:0005516",
  "gene_symbol": "MKNK1",
  "gene": "UniProtKB:Q9BUB5",
  "term_label": "calmodulin binding"
}